phytol metabolic process [GO:0033306] (biological process) Relationships: is a type of diterpenoid metabolic process [GO:0016101]; is a type of primary alcohol metabolic process [GO:0034308]; is a type of fatty alcohol metabolic process [GO:1903173] Sources: GOC:mah Definition: The chemical reactions and pathways involving phytol, (2E,7R,11R)-3,7,11,15-tetramethylhexadec-2-en-1-ol. Subtypes: GO:0033520 Also known as: phytol metabolism